site-specific DNA replication termination [GO:0071170] (biological process) References: PMID:12009298, PMID:18723894 Sources: GOC:mah Definition: A DNA replication termination process that takes place at a specific termination site. Note: See also the biological process term 'replication fork arrest ; GO:0043111' and its children. Subtypes: site-specific DNA replication termination at RTS1 barrier [GO:0071171], cis-acting DNA replication termination [GO:0071946] Relationships: is a type of GO:0006274